{
  "gene_name": "Neuroguidin",
  "gene_symbol": "NGDN",
  "gene": "UniProtKB:Q8NEJ9",
  "term_id": "UNKNOWN:0001",
  "term_label": "Unknown molecular function"
}